positive regulation of presynapse assembly [GO:1905608] (biological process) References: PMID:25533483 Sources: GOC:PARL, GOC:TermGenie, GOC:bc, GO_REF:0000058 Subtypes: positive regulation of presynaptic active zone assembly [GO:1905520] Also known as: positive regulation of presynapse biogenesis, positive regulation of presynaptic terminal assembly, up regulation of presynapse assembly, up regulation of presynapse biogenesis, up regulation of presynaptic terminal assembly, up-regulation of presynapse assembly, up-regulation of presynapse biogenesis, up-regulation of presynaptic terminal assembly, upregulation of presynapse assembly, upregulation of presynapse biogenesis, upregulation of presynaptic terminal assembly, activation of presynapse assembly, activation of presynapse biogenesis, activation of presynaptic terminal assembly Definition: Any process that activates or increases the frequency, rate or extent of presynapse assembly. Relationships: is a type of positive regulation of cellular component organization [GO:0051130]; is a type of GO:1905606; positively regulates presynapse assembly [GO:0099054]